response to heparin [GO:0071503] (biological process) Definition: Any process that results in a change in state or activity of a cell or an organism (in terms of movement, secretion, enzyme production, gene expression, etc.) as a result of a heparin stimulus. Sources: GOC:mah, GOC:yaf Relationships: is a type of response to nitrogen compound [GO:1901698]; is a type of GO:1901700 Subtypes: cellular response to heparin [GO:0071504]